{
  "gene_symbol": "C16orf90",
  "term_label": "Unknown cellular component",
  "gene_name": "Uncharacterized protein C16orf90",
  "gene": "UniProtKB:A8MZG2",
  "term_id": "UNKNOWN:0003"
}